{
  "gene_symbol": "STAT5A",
  "gene": "UniProtKB:P42229",
  "gene_name": "Signal transducer and activator of transcription 5A",
  "term_label": "RNA polymerase II cis-regulatory region sequence-specific DNA binding",
  "term_id": "GO:0000978"
}